{
  "gene_name": "Putative NOL1_NOP2_Sun domain family member 5B",
  "gene": "UniProtKB:Q3KNT7",
  "gene_symbol": "NSUN5P1",
  "term_label": "Unknown molecular function",
  "term_id": "UNKNOWN:0001"
}